negative regulation of mitochondrial transcription [GO:0170070] (biological process) Definition: Any process that stops, prevents, or reduces the frequency, rate or extent of transcription occurring in the mitochondrion. References: PMID:23300484 Relationships: is a type of negative regulation of DNA-templated transcription [GO:0045892]; is a type of regulation of mitochondrial transcription [GO:1903108]; RO_0002212 mitochondrial transcription [GO:0006390]